{
  "gene_symbol": "GPRIN3",
  "term_id": "UNKNOWN:0001",
  "gene": "UniProtKB:Q6ZVF9",
  "term_label": "Unknown molecular function",
  "gene_name": "G protein-regulated inducer of neurite outgrowth 3"
}